{
  "gene": "UniProtKB:O43581",
  "term_id": "GO:0005544",
  "gene_symbol": "SYT7",
  "gene_name": "Synaptotagmin-7",
  "term_label": "calcium-dependent phospholipid binding"
}